{
  "gene_symbol": "USP28",
  "term_id": "GO:0004843",
  "gene": "UniProtKB:Q96RU2",
  "gene_name": "Ubiquitin carboxyl-terminal hydrolase 28",
  "term_label": "cysteine-type deubiquitinase activity"
}